{
  "gene_symbol": "COQ10A",
  "gene_name": "Coenzyme Q-binding protein COQ10 homolog A, mitochondrial",
  "term_id": "UNKNOWN:0001",
  "gene": "UniProtKB:Q96MF6",
  "term_label": "Unknown molecular function"
}